oidium formation [GO:0034297] (BP) Sources: GOC:mah, https://doi.org/10.1007/BF02464287 Relationships: is a type of asexual sporulation [GO:0030436] Definition: The process in which oidia, a type of asexual spore found in fungi, are formed. Oidia are borne a few at a time on very simple hyphae that protrude a short distance into the substrate, and are usually presumed not to constitute the main reproductive strategy of the fungus.